{
  "gene_symbol": "NPM3",
  "term_label": "nucleoplasm",
  "gene": "UniProtKB:O75607",
  "term_id": "GO:0005654",
  "gene_name": "Nucleoplasmin-3"
}